symbiont-mediated perturbation of host NF-kappaB cascade [GO:0085032] (biological process) Definition: A process in which a symbiont alters or subverts an NF-kappaB-mediated signaling cascade in its host organism. The host is defined as the larger of the organisms involved in a symbiotic interaction. Sources: GOC:pamgo_curators Relationships: is a type of symbiont-mediated perturbation of host signal transduction pathway [GO:0052027] Also known as: modulation by symbiont of host NF-kappaB-mediated signal transduction pathway, perturbation of host I-kappaB kinase/NF-kappaB cascade, modulation by symbiont of host I-kappaB kinase/NF-kappaB cascade, perturbation of host canonical NF-kappaB cascade, symbiont-mediated perturbation of host canonical NF-kappaB cascade Subtypes: symbiont-mediated activation of host NF-kappaB cascade [GO:0085033], GO:0085034